regulation of activation of membrane attack complex [GO:0001969] (BP) Subtypes: positive regulation of activation of membrane attack complex [GO:0001970], GO:0001971 Definition: Any process that modulates the frequency, rate or extent of the activation of the membrane attack complex components of the complement cascade. Sources: GOC:hjd Also known as: regulation of MAC assembly, regulation of MAC formation, regulation of activation of MAC, regulation of membrane attack complex assembly, regulation of membrane attack complex formation, regulation of activation of TCC, regulation of activation of terminal complement complex, regulation of activation of the terminal complement cascade Relationships: is a type of regulation of complement activation [GO:0030449]; regulates activation of membrane attack complex [GO:0001905]